RNA nucleotide deletion [GO:0070706] (biological process) Subtypes: RNA uridine deletion [GO:0070710] Sources: GOC:cb, GOC:mah Also known as: RNA nucleotide excision Definition: The modification of an RNA molecule by removal of a single nucleotide. Relationships: is a type of RNA modification [GO:0009451]